cyclic-di-AMP binding [GO:0180001] (molecular function) References: PMID:32843560, PMID:36629470 Also known as: cyclic dimeric adenosine monophosphate binding Definition: Binding to a cyclic di-AMP nucleotide. Relationships: is a type of GO:0030551; is a type of adenyl ribonucleotide binding [GO:0032559]